{
  "term_id": "GO:1903566",
  "gene_name": "Endosome-associated-trafficking regulator 1",
  "term_label": "positive regulation of protein localization to cilium",
  "gene": "UniProtKB:Q96C92",
  "gene_symbol": "ENTR1"
}